{
  "gene_symbol": "PLEKHB2",
  "term_id": "GO:0016020",
  "gene_name": "Pleckstrin homology domain-containing family B member 2",
  "term_label": "membrane",
  "gene": "UniProtKB:Q96CS7"
}